{
  "gene_symbol": "CCDC125",
  "gene_name": "Coiled-coil domain-containing protein 125",
  "gene": "UniProtKB:Q86Z20",
  "term_label": "negative regulation of cell motility",
  "term_id": "GO:2000146"
}